glomerulus development [GO:0032835] (biological process) Definition: The progression of the glomerulus over time from its initial formation until its mature state. The glomerulus is a capillary tuft which forms a close network with the visceral epithelium (podocytes) and the mesangium to form the filtration barrier and is surrounded by Bowman's capsule in nephrons of the vertebrate kidney. The glomerulus is part of the nephron and is restricted to one body segment. Sources: GOC:mah, GOC:mtg_kidney_jan10 Also known as: glomerular development Relationships: is a type of anatomical structure development [GO:0048856]; is part of nephron development [GO:0072006] Subtypes: GO:0039021, mesonephric glomerulus development [GO:0061224], metanephric glomerulus development [GO:0072224] Regulation: regulated by regulation of glomerulus development [GO:0090192]; positively regulated by positive regulation of glomerulus development [GO:0090193]; negatively regulated by negative regulation of glomerulus development [GO:0090194]